maintenance of protein localization to heterochromatin [GO:1990153] (BP) References: PMID:21300781 Also known as: maintenance of protein localisation to heterochromatin, maintenance of protein location in heterochromatin Relationships: is_a GO:0032507; is part of protein localization to heterochromatin [GO:0097355] Definition: A process in which a protein is maintained in a location in telomeric heterochromatin.